{
  "gene_name": "Platelet-derived growth factor receptor-like protein",
  "gene": "UniProtKB:Q15198",
  "term_label": "Unknown cellular component",
  "gene_symbol": "PDGFRL",
  "term_id": "UNKNOWN:0003"
}